{
  "gene_name": "T-cell surface glycoprotein CD3 delta chain",
  "gene": "UniProtKB:P04234",
  "term_id": "GO:0007166",
  "term_label": "cell surface receptor signaling pathway",
  "gene_symbol": "CD3D"
}